{
  "term_id": "GO:0006954",
  "term_label": "inflammatory response",
  "gene_symbol": "CCL5",
  "gene": "UniProtKB:P13501",
  "gene_name": "C-C motif chemokine 5"
}